mammary gland cord elongation [GO:0060654] (biological process) Definition: The process in which the mammary gland sprout grows along its axis. Regulation: RO_0002211 by regulation of mammary gland cord elongation by mammary fat precursor cell-epithelial cell signaling [GO:0060657] References: PMID:12558599 Sources: GOC:dph Relationships: is a type of branch elongation involved in mammary gland duct branching [GO:0060751]; is part of mammary gland cord morphogenesis [GO:0060652]